PLC activating G protein-coupled glutamate receptor activity [GO:0001639] (molecular function) Definition: A G protein-coupled receptor that binds glutamate and is linked to the inositol 1,4,5-trisphosphate/calcium signaling system. References: PMID:9016303 Relationships: is a type of G protein-coupled glutamate receptor activity [GO:0098988]; is part of phospholipase C-activating G protein-coupled glutamate receptor signaling pathway [GO:0007206] Also known as: PLC activating G-protein coupled glutamate receptor activity, PLC activating metabotropic glutamate receptor activity, phospholipase C activating metabotropic glutamate receptor activity, Group I metabotropic glutamate receptor, group I metabotropic glutamate receptor activity